{
  "gene": "UniProtKB:Q8TDD1",
  "gene_name": "ATP-dependent RNA helicase DDX54",
  "term_id": "UNKNOWN:0001",
  "term_label": "Unknown molecular function",
  "gene_symbol": "DDX54"
}